acetoacetic acid catabolic process [GO:0043442] (biological process) Also known as: acetoacetic acid breakdown, acetoacetic acid catabolism, acetoacetic acid degradation Sources: GOC:jl Relationships: is_a short-chain fatty acid catabolic process [GO:0019626]; is a type of GO:0043438; is a type of GO:0046952 Definition: The chemical reactions and pathways resulting in the breakdown of acetoacetic acid, a beta-keto acid of the keto acid group, empirical formula is C4H6O3 or CH3COCH2COOH.